negative regulation of insulin-like growth factor receptor signaling pathway [GO:0043569] (biological process) Also known as: down regulation of insulin-like growth factor receptor signaling pathway, down-regulation of insulin-like growth factor receptor signaling pathway, downregulation of insulin-like growth factor receptor signaling pathway, negative regulation of IGF receptor signaling pathway, negative regulation of IGF receptor signalling pathway, negative regulation of insulin-like growth factor receptor signalling pathway, inhibition of insulin-like growth factor receptor signaling pathway Definition: Any process that stops, prevents, or reduces the frequency, rate or extent of insulin-like growth factor receptor signaling. Sources: GOC:bf Relationships: is a type of negative regulation of signal transduction [GO:0009968]; is_a regulation of insulin-like growth factor receptor signaling pathway [GO:0043567]; RO_0002212 GO:0048009